{
  "gene": "UniProtKB:Q96NU7",
  "term_label": "imidazolonepropionase activity",
  "gene_symbol": "AMDHD1",
  "gene_name": "Probable imidazolonepropionase",
  "term_id": "GO:0050480"
}